GDP-4-dehydro-6-deoxy-D-mannose-4-aminotransferase activity [GO:0102933] (molecular function) Sources: GOC:pz, RHEA:36779 Definition: Catalysis of the reaction: GDP-4-amino-4,6-dideoxy-alpha-D-mannose + 2-oxoglutarate = GDP-4-dehydro-6-deoxy-alpha-D-mannose + L-glutamate. Relationships: is a type of transaminase activity [GO:0008483]